type 1 metabotropic GABA receptor binding [GO:0031796] (molecular function) Relationships: is a type of G protein-coupled GABA receptor binding [GO:0031795] Sources: GOC:mah, GOC:nln Definition: Binding to a type 1 metabotropic GABA receptor. Also known as: type 1 metabotropic GABA receptor ligand